{
  "term_label": "synaptic transmission, glutamatergic",
  "gene_symbol": "UNC13B",
  "gene_name": "Protein unc-13 homolog B",
  "term_id": "GO:0035249",
  "gene": "UniProtKB:O14795"
}